{
  "gene_symbol": "TRBV28",
  "term_label": "cell surface receptor signaling pathway",
  "term_id": "GO:0007166",
  "gene_name": "T cell receptor beta variable 28",
  "gene": "UniProtKB:A0A5B6"
}